FtsQBL complex [GO:1990587] (cellular component) Definition: A protein complex required for prokaryotic cell division (FtsZ-dependent cytokinesis). Part of the divisome. Assembled independently of the other divisome components in the cytoplasm prior to transport to the cell septum. In E. coli consists of FtsB, FtsL and FtsQ. References: PMID:15165235, PMID:21784946 Sources: GOC:bhm Also known as: FtsB-FtsL-FtsQ complex Note: An example of this is FtsB in E. coli (P0A6S5) in PMID:15165235 (inferred from physical interaction). Relationships: is a type of divisome complex [GO:1990586]